{
  "term_label": "vesicle fusion",
  "gene": "UniProtKB:Q13190",
  "gene_name": "Syntaxin-5",
  "gene_symbol": "STX5",
  "term_id": "GO:0006906"
}